{
  "gene_symbol": "ZNF678",
  "term_label": "regulation of DNA-templated transcription",
  "gene_name": "Zinc finger protein 678",
  "gene": "UniProtKB:Q5SXM1",
  "term_id": "GO:0006355"
}